{
  "gene": "UniProtKB:P15884",
  "term_label": "RNA polymerase II cis-regulatory region sequence-specific DNA binding",
  "gene_name": "Transcription factor 4",
  "term_id": "GO:0000978",
  "gene_symbol": "TCF4"
}